{
  "gene_name": "Tyrosine--tRNA ligase, cytoplasmic",
  "term_id": "UNKNOWN:0003",
  "gene": "UniProtKB:P54577",
  "gene_symbol": "YARS1",
  "term_label": "Unknown cellular component"
}